{
  "gene_symbol": "CHCHD2P9",
  "gene_name": "Putative coiled-coil-helix-coiled-coil-helix domain-containing protein CHCHD2P9, mitochondrial",
  "gene": "UniProtKB:Q5T1J5",
  "term_id": "GO:0045944",
  "term_label": "positive regulation of transcription by RNA polymerase II"
}